{
  "gene": "UniProtKB:Q9NRL2",
  "gene_name": "Bromodomain adjacent to zinc finger domain protein 1A",
  "term_id": "GO:0006355",
  "term_label": "regulation of DNA-templated transcription",
  "gene_symbol": "BAZ1A"
}